4-hydroxyquinoline 3-monooxygenase activity [GO:0047093] (molecular function) Sources: EC:1.14.13.62, RHEA:19325 Also known as: 1-H-4-oxoquinoline 3-monooxygenase activity, quinolin-4(1H)-one 3-monooxygenase activity, quinolin-4(1H)-one,NADH:oxygen oxidoreductase (3-oxygenating) Definition: Catalysis of the reaction: H+ + NADH + O2 + quinolin-4-ol = H2O + NAD+ + quinoline-3,4-diol. Relationships: is_a oxidoreductase activity, acting on paired donors, with incorporation or reduction of molecular oxygen, NAD(P)H as one donor, and incorporation of one atom of oxygen [GO:0016709]